negative regulation of development of symbiont in host [GO:0044131] (biological process) Note: This term partially replaces the obsolete term 'negative regulation of growth or development of symbiont in host ; GO:0033667'. See also 'negative regulation of growth of symbiont in host ; GO:0044130'. Relationships: is a type of regulation of development of symbiont in host [GO:0044127]; is a type of GO:0044147; negatively regulates development of symbiont in host [GO:0044114] Sources: GOC:jl, GOC:pamgo_curators Definition: Any process in which the symbiont stops, prevents or reduces its progression from an initial condition to a later condition, within the cells or tissues of the host organism. The host is defined as the larger of the organisms involved in the symbiotic interaction.